{
  "gene_name": "DnaJ homolog subfamily C member 24",
  "gene_symbol": "DNAJC24",
  "gene": "UniProtKB:Q6P3W2",
  "term_id": "GO:0008198",
  "term_label": "ferrous iron binding"
}